{
  "gene": "UniProtKB:Q96A70",
  "gene_name": "Antizyme inhibitor 2",
  "gene_symbol": "AZIN2",
  "term_id": "GO:1902269",
  "term_label": "positive regulation of polyamine transmembrane transport"
}